{
  "gene_symbol": "PARVG",
  "gene_name": "Gamma-parvin",
  "term_id": "GO:0005925",
  "gene": "UniProtKB:Q9HBI0",
  "term_label": "focal adhesion"
}